{
  "gene_name": "WD repeat domain phosphoinositide-interacting protein 4",
  "gene_symbol": "WDR45",
  "term_id": "GO:0000422",
  "gene": "UniProtKB:Q9Y484",
  "term_label": "autophagy of mitochondrion"
}